chlorophyll biosynthetic process [GO:0015995] (biological process) Also known as: chlorophyll anabolism, chlorophyll biosynthesis, chlorophyll formation, chlorophyll synthesis Sources: GOC:jl Relationships: is a type of GO:0006779; is_a chlorophyll metabolic process [GO:0015994]; is a type of pigment biosynthetic process [GO:0046148] Subtypes: bacteriochlorophyll biosynthetic process [GO:0030494], chlorophyll a biosynthetic process [GO:0033305], light-dependent chlorophyll biosynthetic process [GO:0036067], light-independent chlorophyll biosynthetic process [GO:0036068] Regulation: regulated by regulation of chlorophyll biosynthetic process [GO:0010380]; negatively regulated by negative regulation of chlorophyll biosynthetic process [GO:1902325]; positively regulated by GO:1902326 Definition: The chemical reactions and pathways resulting in the formation of chlorophyll, any compound of magnesium complexed in a porphyrin (tetrapyrrole) ring and which functions as a photosynthetic pigment, from less complex precursors.